{
  "gene_symbol": "ADGRD1",
  "gene_name": "Adhesion G-protein coupled receptor D1",
  "term_id": "GO:0007189",
  "term_label": "adenylate cyclase-activating G protein-coupled receptor signaling pathway",
  "gene": "UniProtKB:Q6QNK2"
}